{
  "gene": "UniProtKB:Q6AI12",
  "term_id": "UNKNOWN:0001",
  "gene_symbol": "ANKRD40",
  "term_label": "Unknown molecular function",
  "gene_name": "Ankyrin repeat domain-containing protein 40"
}